{
  "term_label": "fibroblast growth factor binding",
  "gene_name": "Fibroblast growth factor receptor 4",
  "term_id": "GO:0017134",
  "gene_symbol": "FGFR4",
  "gene": "UniProtKB:P22455"
}